{
  "gene_symbol": "IFT25",
  "gene_name": "Intraflagellar transport protein 25 homolog",
  "term_label": "smoothened signaling pathway",
  "gene": "UniProtKB:Q9Y547",
  "term_id": "GO:0007224"
}